myofibril assembly [GO:0030239] (biological process) Sources: GOC:mah Subtypes: skeletal myofibril assembly [GO:0014866], cardiac myofibril assembly [GO:0055003] Definition: Formation of myofibrils, the repeating units of striated muscle. Relationships: is a type of cellular component assembly involved in morphogenesis [GO:0010927]; is a type of actomyosin structure organization [GO:0031032]; is_a supramolecular fiber organization [GO:0097435]; is a type of membraneless organelle assembly [GO:0140694]; is part of striated muscle cell development [GO:0055002]